{
  "term_label": "endoplasmic reticulum membrane",
  "term_id": "GO:0005789",
  "gene_name": "E3 UFM1-protein ligase 1",
  "gene_symbol": "UFL1",
  "gene": "UniProtKB:O94874"
}